{
  "term_label": "Unknown molecular function",
  "gene": "UniProtKB:Q68CL5",
  "term_id": "UNKNOWN:0001",
  "gene_symbol": "TPGS2",
  "gene_name": "Tubulin polyglutamylase complex subunit 2"
}